regulation of relaxation of cardiac muscle [GO:1901897] (biological process) Definition: Any process that modulates the frequency, rate or extent of relaxation of cardiac muscle. Relationships: is_a regulation of relaxation of muscle [GO:1901077]; regulates relaxation of cardiac muscle [GO:0055119] References: PMID:19708671 Sources: GOC:BHF, GOC:TermGenie, GOC:rl Subtypes: negative regulation of relaxation of cardiac muscle [GO:1901898], positive regulation of relaxation of cardiac muscle [GO:1901899]